{
  "term_id": "GO:0010468",
  "gene_name": "Sonic hedgehog protein",
  "gene_symbol": "SHH",
  "gene": "UniProtKB:Q15465",
  "term_label": "regulation of gene expression"
}